prospore septin filament array [GO:0032165] (cellular component) References: PMID:16151244 Sources: GOC:krc Definition: Arrays of septin filaments, or bars, found in a series of filamentous structures; observed in the prospore membrane during spore formation. Relationships: is a type of septin filament array [GO:0032160]